chondroitin-glucuronate 5-epimerase activity [GO:0047757] (molecular function) Also known as: chondroitin D-glucuronosyl 5-epimerase activity, chondroitin-D-glucuronate 5-epimerase activity, dermatan-sulfate 5-epimerase activity, polyglucuronate 5-epimerase activity, urunosyl C-5 epimerase activity Relationships: is a type of racemase and epimerase activity, acting on carbohydrates and derivatives [GO:0016857] Sources: EC:5.1.3.19, MetaCyc:CHONDROITIN-GLUCURONATE-5-EPIMERASE-RXN Definition: Catalysis of the reaction: chondroitin D-glucuronate = dermatan L-iduronate.